astaxanthin biosynthetic process [GO:1901815] (biological process) References: PMID:16434154 Sources: GOC:TermGenie, GOC:yaf, MetaCyc:PWY-5288, UniPathway:UPA00387 Definition: The chemical reactions and pathways resulting in the formation of astaxanthin. Relationships: is a type of xanthophyll biosynthetic process [GO:0016123] Also known as: astaxanthin anabolism, astaxanthin biosynthesis, astaxanthin formation, astaxanthin synthesis